{
  "term_id": "GO:0001228",
  "term_label": "DNA-binding transcription activator activity, RNA polymerase II-specific",
  "gene_symbol": "MEIS3P2",
  "gene_name": "Putative homeobox protein Meis3-like 2",
  "gene": "UniProtKB:A8K0S8"
}